{
  "gene": "UniProtKB:A0A0C4DH55",
  "term_id": "UNKNOWN:0001",
  "term_label": "Unknown molecular function",
  "gene_symbol": "IGKV3D-7",
  "gene_name": "Immunoglobulin kappa variable 3D-7"
}